positive regulation of melanization defense response [GO:0035008] (biological process) Also known as: positive regulation of melanization defence response, up regulation of melanization defense response, up-regulation of melanization defense response, upregulation of melanization defense response, activation of melanization defense response, stimulation of melanization defense response Definition: Any process that increases the rate or extent of the melanization defense response during injury or invasion. Relationships: is a type of positive regulation of metabolic process [GO:0009893]; is a type of regulation of melanization defense response [GO:0035007]; is_a positive regulation of innate immune response [GO:0045089]; RO_0002213 GO:0035006 Sources: GOC:bf